{
  "term_label": "positive regulation of natural killer cell mediated cytotoxicity",
  "gene_symbol": "KLRK1",
  "term_id": "GO:0045954",
  "gene_name": "NKG2-D type II integral membrane protein",
  "gene": "UniProtKB:P26718"
}